{
  "gene": "UniProtKB:Q9H195",
  "term_id": "UNKNOWN:0001",
  "gene_name": "Mucin-3B",
  "term_label": "Unknown molecular function",
  "gene_symbol": "MUC3B"
}